{
  "gene_name": "Inositol 1,4,5-triphosphate receptor associated 1",
  "gene": "UniProtKB:Q9Y6F6",
  "term_label": "Unknown molecular function",
  "term_id": "UNKNOWN:0001",
  "gene_symbol": "IRAG1"
}